{
  "gene": "UniProtKB:Q07011",
  "gene_name": "Tumor necrosis factor receptor superfamily member 9",
  "term_label": "signaling receptor activity",
  "term_id": "GO:0038023",
  "gene_symbol": "TNFRSF9"
}